formation of anatomical boundary [GO:0048859] (biological process) Subtypes: formation of animal organ boundary [GO:0010160], GO:0021547, rhombomere boundary formation [GO:0021654], forebrain-midbrain boundary formation [GO:0021905], hindbrain-spinal cord boundary formation [GO:0021906], zona limitans intrathalamica formation [GO:0022006], equator specification [GO:0045317], GO:0060288, formation of plant organ boundary [GO:0090691] Relationships: is a type of anatomical structure formation involved in morphogenesis [GO:0048646] Definition: The process in which the limits of an anatomical structure are generated. An anatomical structure is any biological entity that occupies space and is distinguished from its surroundings. Anatomical structures can be macroscopic such as a carpel, or microscopic such as an acrosome. Sources: GO_REF:0000021